{
  "term_label": "retinal metabolic process",
  "gene": "UniProtKB:Q8N3Y7",
  "term_id": "GO:0042574",
  "gene_symbol": "SDR16C5",
  "gene_name": "Epidermal retinol dehydrogenase 2"
}